{
  "term_id": "GO:0003729",
  "term_label": "mRNA binding",
  "gene_name": "Nuclear inhibitor of protein phosphatase 1",
  "gene": "UniProtKB:Q12972",
  "gene_symbol": "PPP1R8"
}